{
  "gene": "UniProtKB:A6NKF2",
  "gene_symbol": "ARID3C",
  "term_id": "GO:0003677",
  "gene_name": "AT-rich interactive domain-containing protein 3C",
  "term_label": "DNA binding"
}